{
  "term_id": "UNKNOWN:0003",
  "gene": "UniProtKB:A0A1B0GTR4",
  "term_label": "Unknown cellular component",
  "gene_name": "Putative small proline-rich protein 5",
  "gene_symbol": "SPRR5"
}